{
  "gene": "UniProtKB:P04233",
  "term_label": "T cell activation involved in immune response",
  "gene_name": "HLA class II histocompatibility antigen gamma chain",
  "term_id": "GO:0002286",
  "gene_symbol": "CD74"
}